{
  "term_label": "Unknown molecular function",
  "gene_symbol": "A0A0G2JKW9",
  "gene_name": "Uncharacterized protein",
  "term_id": "UNKNOWN:0001",
  "gene": "UniProtKB:A0A0G2JKW9"
}